neural crest cell migration involved in autonomic nervous system development [GO:1901166] (biological process) Relationships: is a type of neural crest cell migration [GO:0001755]; is part of autonomic nervous system development [GO:0048483] Sources: GOC:BHF, GOC:TermGenie Subtypes: GO:1903045 Definition: Any neural crest cell migration that is involved in autonomic nervous system development.